tRNA (guanine(46)-N7)-methyltransferase activity [GO:0008176] (molecular function) Definition: Catalysis of the reaction: guanosine46 in tRNA + S-adenosyl-L-methionine = N7-methylguanosine46 in tRNA + S-adenosyl-L-homocysteine. Sources: RHEA:42708 Also known as: 7-methylguanine transfer ribonucleate methylase activity, N7-methylguanine methylase activity, tRNA (guanine-N7-)-methyltransferase activity, tRNA guanine 7-methyltransferase activity, tRNA (guanine(46)-N7-)-methyltransferase activity, tRNA (guanosine(46)-N(7))-methyltransferase activity, tRNA (guanosine(46)-N7)-methyltransferase activity, tRNA (guanosine(46)-N7-)-methyltransferase activity Relationships: is a type of tRNA (guanine) methyltransferase activity [GO:0016423]; is part of tRNA (guanine-N7)-methylation [GO:0106004]